{
  "gene_symbol": "KLHDC7B",
  "term_label": "Unknown biological process",
  "gene_name": "Kelch domain-containing protein 7B",
  "term_id": "UNKNOWN:0002",
  "gene": "UniProtKB:Q96G42"
}